{
  "gene_name": "Prosaposin receptor GPR37",
  "term_label": "G protein-coupled peptide receptor activity",
  "term_id": "GO:0008528",
  "gene": "UniProtKB:O15354",
  "gene_symbol": "GPR37"
}